{
  "term_id": "UNKNOWN:0003",
  "term_label": "Unknown cellular component",
  "gene_symbol": "NPS",
  "gene_name": "Neuropeptide S",
  "gene": "UniProtKB:P0C0P6"
}